commitment of multipotent stem cells to neuronal lineage in forebrain [GO:0021898] (biological process) Definition: The initial commitment of cells whereby the developmental fate of a cell becomes restricted such that it will develop into some type of neuron in the forebrain. Relationships: is a type of GO:0021877 References: PMID:12626695 Sources: GOC:cls, GOC:dgh, GOC:dph, GOC:jid, GO_REF:0000021 Subtypes: ventricular zone cell fate commitment [GO:0021900], early neuron fate commitment in forebrain [GO:0021901], radial glial cell fate commitment in forebrain [GO:0022023]